{
  "term_label": "cAMP-dependent protein kinase activity",
  "gene_name": "cAMP-dependent protein kinase catalytic subunit alpha",
  "term_id": "GO:0004691",
  "gene": "UniProtKB:P17612",
  "gene_symbol": "PRKACA"
}